{
  "gene": "UniProtKB:Q8IYK2",
  "term_label": "Unknown cellular component",
  "gene_symbol": "CCDC105",
  "gene_name": "Coiled-coil domain-containing protein 105",
  "term_id": "UNKNOWN:0003"
}